{
  "term_label": "UDP-N-acetylgalactosamine transmembrane transporter activity",
  "gene_symbol": "SLC35D2",
  "gene": "UniProtKB:Q76EJ3",
  "gene_name": "UDP-N-acetylglucosamine_UDP-glucose_GDP-mannose transporter",
  "term_id": "GO:0005463"
}